{
  "gene": "UniProtKB:P36954",
  "term_label": "transcription-coupled nucleotide-excision repair",
  "term_id": "GO:0006283",
  "gene_symbol": "POLR2I",
  "gene_name": "DNA-directed RNA polymerase II subunit RPB9"
}